{
  "term_label": "Unknown cellular component",
  "term_id": "UNKNOWN:0003",
  "gene": "UniProtKB:P0DP06",
  "gene_symbol": "IGHV4-30-4",
  "gene_name": "Immunoglobulin heavy variable 4-30-4"
}